{
  "gene_symbol": "MYSM1",
  "term_id": "GO:0045944",
  "term_label": "positive regulation of transcription by RNA polymerase II",
  "gene": "UniProtKB:Q5VVJ2",
  "gene_name": "Deubiquitinase MYSM1"
}